{
  "term_id": "GO:0000978",
  "gene_name": "Nuclear receptor subfamily 2 group C member 1",
  "gene_symbol": "NR2C1",
  "term_label": "RNA polymerase II cis-regulatory region sequence-specific DNA binding",
  "gene": "UniProtKB:P13056"
}